{
  "gene": "UniProtKB:Q32NB8",
  "term_label": "mitochondrion",
  "gene_symbol": "PGS1",
  "gene_name": "CDP-diacylglycerol--glycerol-3-phosphate 3-phosphatidyltransferase, mitochondrial",
  "term_id": "GO:0005739"
}